{
  "gene": "UniProtKB:Q08170",
  "gene_symbol": "SRSF4",
  "gene_name": "Serine_arginine-rich splicing factor 4",
  "term_label": "mRNA binding",
  "term_id": "GO:0003729"
}